{
  "gene_symbol": "IL1A",
  "term_label": "positive regulation of immature T cell proliferation in thymus",
  "gene_name": "Interleukin-1 alpha",
  "term_id": "GO:0033092",
  "gene": "UniProtKB:P01583"
}